{
  "gene_symbol": "RFC5",
  "term_label": "nucleus",
  "gene_name": "Replication factor C subunit 5",
  "gene": "UniProtKB:P40937",
  "term_id": "GO:0005634"
}